tartrate:succinate antiporter activity [GO:0015516] (molecular function) Relationships: is a type of succinate transmembrane transporter activity [GO:0015141]; is a type of antiporter activity [GO:0015297]; is a type of tartrate transmembrane transporter activity [GO:0015554] Definition: Enables the transfer of a solute or solutes from one side of a membrane to the other according to the reaction: tartrate(out) + succinate(in) = tartrate(in) + succinate(out). Sources: TC:2.A.47.3.3